versiconal reductase activity [GO:0102976] (molecular function) Relationships: is a type of GO:0016616 Sources: RHEA:35699 Definition: Catalysis of the reaction: (2S)-versicolorone + NADP+ = 1'-hydroxyversicolorone + H+ + NADPH.